leukotriene production involved in inflammatory response [GO:0002540] (biological process) Definition: The synthesis or release of any leukotriene following a stimulus as part of an inflammatory response, resulting in an increase in its intracellular or extracellular levels. Sources: GOC:add, ISBN:0781735149 Also known as: leukotriene production involved in acute inflammatory response Relationships: is a type of GO:0002538 Regulation: regulated by regulation of leukotriene production involved in inflammatory response [GO:0035490]; positively regulated by positive regulation of leukotriene production involved in inflammatory response [GO:0035491]; negatively regulated by negative regulation of leukotriene production involved in inflammatory response [GO:0035492]